{
  "gene": "UniProtKB:P05423",
  "term_id": "GO:0042797",
  "term_label": "tRNA transcription by RNA polymerase III",
  "gene_symbol": "POLR3D",
  "gene_name": "DNA-directed RNA polymerase III subunit RPC4"
}